{
  "gene_symbol": "PBX3",
  "gene_name": "Pre-B-cell leukemia transcription factor 3",
  "term_label": "neuron development",
  "term_id": "GO:0048666",
  "gene": "UniProtKB:P40426"
}